{
  "gene": "UniProtKB:Q01130",
  "term_id": "GO:0000381",
  "gene_symbol": "SRSF2",
  "term_label": "regulation of alternative mRNA splicing, via spliceosome",
  "gene_name": "Serine_arginine-rich splicing factor 2"
}